peptidyl-serine phosphopantetheinylation [GO:0018070] (biological process) Sources: RESID:AA0150 Relationships: is a type of peptidyl-serine modification [GO:0018209]; is a type of GO:0018215 Definition: The phosphopantetheinylation of peptidyl-serine to form peptidyl-O-phosphopantetheine-L-serine.